{
  "term_id": "GO:0010975",
  "gene": "UniProtKB:P49840",
  "term_label": "regulation of neuron projection development",
  "gene_name": "Glycogen synthase kinase-3 alpha",
  "gene_symbol": "GSK3A"
}